pyridoxamine transmembrane transporter activity [GO:0031927] (molecular function) Definition: Enables the transfer of pyridoxamine from one side of a membrane to the other. Pyridoxamine, 4-(aminomethyl)-5-(hydroxymethyl)-2-methylpyridin-3-ol, is one of the vitamin B6 compounds. Pyridoxal, pyridoxamine and pyridoxine are collectively known as vitamin B6, and are efficiently converted to the biologically active form of vitamin B6, pyridoxal phosphate. Sources: GOC:mah Relationships: is a type of transmembrane transporter activity [GO:0022857]; is part of GO:1903091